cellular response to cytochalasin B [GO:0072749] (biological process) Sources: GOC:mah Definition: Any process that results in a change in state or activity of a cell (in terms of movement, secretion, enzyme production, gene expression, etc.) as a result of a cytochalasin B stimulus. Relationships: is a type of response to cytochalasin B [GO:1901328]; is a type of cellular response to nitrogen compound [GO:1901699]; is a type of GO:1901701